oxidoreductase activity, acting on the aldehyde or oxo group of donors [GO:0016903] (molecular function) Definition: Catalysis of an oxidation-reduction (redox) reaction in which an aldehyde or ketone (oxo) group acts as a hydrogen or electron donor and reduces a hydrogen or electron acceptor. Relationships: is a type of oxidoreductase activity [GO:0016491] Subtypes: GO:0016620, GO:0016622, GO:0016623, oxidoreductase activity, acting on the aldehyde or oxo group of donors, disulfide as acceptor [GO:0016624], oxidoreductase activity, acting on the aldehyde or oxo group of donors, iron-sulfur protein as acceptor [GO:0016625], GO:0018493, aldehyde dehydrogenase (FAD-independent) activity [GO:0033727], glyceraldehyde oxidoreductase activity [GO:0043795], GO:0047113, carboxylate reductase activity [GO:0047770], formaldehyde dismutase activity [GO:0047895], alpha-keto amide reductase activity [GO:0051268], GO:0052738 Sources: GOC:ai Also known as: oxidoreductase activity, acting on the aldehyde or oxo group of donors, other acceptors